{
  "gene_name": "Alpha-2-macroglobulin",
  "term_id": "UNKNOWN:0002",
  "term_label": "Unknown biological process",
  "gene_symbol": "A2M",
  "gene": "UniProtKB:P01023"
}